polypeptide conformation or assembly isomerase activity [GO:0120544] (molecular function) Sources: EC:5.6.1.- Subtypes: microfilament motor activity [GO:0000146], microtubule motor activity [GO:0003777], intracellularly ATP-gated chloride channel activity [GO:0005260], microtubule severing ATPase activity [GO:0008568], proteasome-activating activity [GO:0036402] Definition: Catalysis of a reaction that alters the conformation or assembly of a polypeptide. Relationships: is a type of macromolecular conformation isomerase activity [GO:0120543]